Kv4.2-Kv4.3 channel complex [GO:0071197] (cellular component) Relationships: is a type of GO:0008076 Definition: A voltage-gated potassium channel complex that contains the Kv alpha subunits 4.2 and 4.3. References: PMID:15356203